positive regulation of growth of unicellular organism as a thread of attached cells [GO:0070786] (biological process) Sources: GOC:mah Relationships: is a type of regulation of growth of unicellular organism as a thread of attached cells [GO:0070784]; is a type of positive regulation of filamentous growth of a population of unicellular organisms [GO:1900430]; positively regulates growth of unicellular organism as a thread of attached cells [GO:0070783] Subtypes: positive regulation of invasive growth in response to glucose limitation [GO:2000219], positive regulation of pseudohyphal growth [GO:2000222] Definition: Any process that activates or increases the frequency, rate or extent of the process in which cells remain attached after division and form thread-like filaments that may penetrate into a solid growth medium.